{
  "term_label": "extracellular space",
  "gene": "UniProtKB:P03952",
  "gene_symbol": "KLKB1",
  "term_id": "GO:0005615",
  "gene_name": "Plasma kallikrein"
}